{
  "gene": "UniProtKB:P34969",
  "term_label": "G protein-coupled receptor signaling pathway, coupled to cyclic nucleotide second messenger",
  "term_id": "GO:0007187",
  "gene_symbol": "HTR7",
  "gene_name": "5-hydroxytryptamine receptor 7"
}